5-oxoprolinase (ATP-hydrolyzing) activity [GO:0017168] (molecular function) Also known as: 5-OPase activity, 5-oxo-L-prolinase activity, 5-oxo-L-proline amidohydrolase (ATP-hydrolysing), 5-oxoprolinase (ATP-hydrolysing), 5-oxoprolinase activity, L-pyroglutamate hydrolase activity, oxoprolinase activity, pyroglutamase (ATP-hydrolysing), pyroglutamase (ATP-hydrolyzing) activity, pyroglutamase activity, pyroglutamate hydrolase activity, pyroglutamic hydrolase activity Sources: EC:3.5.2.9, RHEA:10348 Relationships: is a type of GO:0016812 Definition: Catalysis of the reaction: 5-oxo-L-proline + ATP + 2 H2O = L-glutamate + ADP + 2 H+ + phosphate.